regulation of transforming growth factor beta receptor signaling pathway [GO:0017015] (biological process) Also known as: regulation of TGF-beta receptor signaling pathway, regulation of TGFbeta receptor signaling pathway, regulation of transforming growth factor beta receptor signalling pathway Sources: GOC:mah Relationships: is a type of GO:0090092; is a type of GO:1903844; regulates GO:0007179 Subtypes: positive regulation of transforming growth factor beta receptor signaling pathway [GO:0030511], negative regulation of transforming growth factor beta receptor signaling pathway [GO:0030512] Definition: Any process that modulates the frequency, rate or extent of activity of any TGF-beta receptor signaling pathway.